{
  "gene_symbol": "RUNX2",
  "term_label": "neuron differentiation",
  "gene_name": "Runt-related transcription factor 2",
  "gene": "UniProtKB:Q13950",
  "term_id": "GO:0030182"
}